{
  "gene_name": "Intraflagellar transport protein 20 homolog",
  "gene": "UniProtKB:Q8IY31",
  "gene_symbol": "IFT20",
  "term_label": "protein localization to cilium",
  "term_id": "GO:0061512"
}